regulation of chemotaxis to arachidonate [GO:1904552] (biological process) Subtypes: negative regulation of chemotaxis to arachidonate [GO:1904553], positive regulation of chemotaxis to arachidonate [GO:1904554] References: PMID:16382163 Sources: GOC:TermGenie, GO_REF:0000058 Definition: Any process that modulates the frequency, rate or extent of chemotaxis to arachidonic acid. Also known as: regulation of chemotaxis to arachidonic acid Relationships: is a type of regulation of chemotaxis [GO:0050920]; regulates GO:0034670